salicylic acid glucosyltransferase (ester-forming) activity [GO:0052639] (molecular function) Also known as: salicylic acid glucosyltransferase activity, UDP:glucose:2-hydroxybenzoic acid glucosyltransferase (ester-forming) activity, UDP:glucose:SA glucosyltransferase (ester-forming) activity, UDP:glucose:salicylate glucosyltransferase (ester-forming) activity, UDP:glucose:salicylic acid glucosyltransferase (ester-forming) activity Sources: MetaCyc:RXN-11659, RHEA:62316 Relationships: is a type of UDP-glucosyltransferase activity [GO:0035251] Definition: Catalysis of the reaction: salicylic acid + UDP-glucose = salicylic acid glucose ester + UDP.